{
  "gene_symbol": "ARFRP1",
  "gene_name": "ADP-ribosylation factor-related protein 1",
  "term_id": "GO:0034067",
  "gene": "UniProtKB:Q13795",
  "term_label": "protein localization to Golgi apparatus"
}